{
  "gene": "UniProtKB:O00712",
  "gene_name": "Nuclear factor 1 B-type",
  "gene_symbol": "NFIB",
  "term_id": "GO:0000981",
  "term_label": "DNA-binding transcription factor activity, RNA polymerase II-specific"
}